{
  "term_label": "Unknown biological process",
  "gene_symbol": "SLX4IP",
  "gene": "UniProtKB:Q5VYV7",
  "term_id": "UNKNOWN:0002",
  "gene_name": "Protein SLX4IP"
}